{
  "term_label": "ubiquitin-like ligase-substrate adaptor activity",
  "gene": "UniProtKB:Q8WZ60",
  "gene_name": "Kelch-like protein 6",
  "gene_symbol": "KLHL6",
  "term_id": "GO:1990756"
}